{
  "term_label": "GTPase activator activity",
  "term_id": "GO:0005096",
  "gene_name": "Phosphatidylinositol 3,4,5-trisphosphate-dependent Rac exchanger 1 protein",
  "gene_symbol": "PREX1",
  "gene": "UniProtKB:Q8TCU6"
}